protein-DNA complex [GO:0032993] (cellular component) Definition: A macromolecular complex containing both protein and DNA molecules. Sources: GOC:mah Also known as: DNA-protein complex Note: Note that this term is intended to classify complexes that have DNA as one of the members of the complex, that is, the complex does not exist if DNA is not present. Protein complexes that interact with DNA e.g. transcription factor complexes should not be classified here. Relationships: is a type of protein-containing complex [GO:0032991] Subtypes: telomere cap complex [GO:0000782], nucleosome [GO:0000786], replisome [GO:0030894], DNA replication preinitiation complex [GO:0031261], enhanceosome [GO:0034206], pre-replicative complex [GO:0036387], retroviral intasome [GO:0044834], telomere-telomerase complex [GO:0070565], DNA recombinase complex [GO:0097519], nucleotide-excision repair, preincision complex [GO:0097520], GO:0097522, transcription preinitiation complex [GO:0097550], GO:1990077, SeqA-DNA complex [GO:1990097], IHF-DNA complex [GO:1990177], HU-DNA complex [GO:1990178]